{
  "gene_symbol": "DUSP8",
  "gene": "UniProtKB:Q13202",
  "gene_name": "Dual specificity protein phosphatase 8",
  "term_id": "GO:0033550",
  "term_label": "MAP kinase tyrosine phosphatase activity"
}